ovulation [GO:0030728] (biological process) Definition: The release of a mature ovum/oocyte from an ovary. Relationships: is a type of GO:0048609; is part of female gamete generation [GO:0007292] Sources: GOC:bf, ISBN:0878932437 Subtypes: GO:0001542 Regulation: regulated by regulation of ovulation [GO:0060278]; positively regulated by GO:0060279; negatively regulated by negative regulation of ovulation [GO:0060280]